{
  "gene": "UniProtKB:Q8WYP3",
  "gene_symbol": "RIN2",
  "term_id": "GO:0030139",
  "term_label": "endocytic vesicle",
  "gene_name": "Ras and Rab interactor 2"
}